{
  "gene_symbol": "TINAGL1",
  "gene_name": "Tubulointerstitial nephritis antigen-like",
  "term_id": "GO:0005764",
  "term_label": "lysosome",
  "gene": "UniProtKB:Q9GZM7"
}